{
  "gene_symbol": "SDC2",
  "gene": "UniProtKB:P34741",
  "gene_name": "Syndecan-2",
  "term_label": "cell migration",
  "term_id": "GO:0016477"
}